{
  "term_label": "plasma membrane",
  "gene_name": "Olfactory receptor 2T1",
  "gene": "UniProtKB:O43869",
  "gene_symbol": "OR2T1",
  "term_id": "GO:0005886"
}